positive regulation of determination of dorsal identity [GO:2000017] (biological process) Sources: GOC:obol Also known as: positive regulation of determination of adaxial identity Relationships: is_a positive regulation of developmental process [GO:0051094]; is_a GO:0051240; is a type of GO:2000015; positively regulates determination of dorsal identity [GO:0048263] Definition: Any process that activates or increases the frequency, rate or extent of determination of dorsal identity.